{
  "gene_name": "TRAF-interacting protein with FHA domain-containing protein A",
  "term_id": "GO:0045087",
  "gene": "UniProtKB:Q96CG3",
  "term_label": "innate immune response",
  "gene_symbol": "TIFA"
}